{
  "gene": "UniProtKB:Q9H6I2",
  "term_label": "endoderm formation",
  "gene_name": "Transcription factor SOX-17",
  "term_id": "GO:0001706",
  "gene_symbol": "SOX17"
}